{
  "gene_symbol": "AFP",
  "gene_name": "Alpha-fetoprotein",
  "gene": "UniProtKB:P02771",
  "term_id": "GO:0031667",
  "term_label": "response to nutrient levels"
}